{
  "gene_name": "Ubiquitin-associated and SH3 domain-containing protein B",
  "term_id": "GO:0004725",
  "term_label": "protein tyrosine phosphatase activity",
  "gene_symbol": "UBASH3B",
  "gene": "UniProtKB:Q8TF42"
}